{
  "gene_name": "UMP-CMP kinase",
  "gene": "UniProtKB:P30085",
  "term_id": "GO:0006225",
  "term_label": "UDP biosynthetic process",
  "gene_symbol": "CMPK1"
}